regulation of nematode larval development [GO:0061062] (biological process) Sources: GOC:dph, GOC:kmv Relationships: is a type of regulation of post-embryonic development [GO:0048580]; regulates GO:0002119 Definition: Any process that modulates the rate, frequency, or extent of nematode larval development, the process whose specific outcome is the progression of the nematode larva over time, from its formation to the mature structure. Nematode larval development begins with the newly hatched first-stage larva (L1) and ends with the end of the last larval stage (for example the fourth larval stage (L4) in C. elegans). Each stage of nematode larval development is characterized by proliferation of specific cell lineages and an increase in body size without alteration of the basic body plan. Nematode larval stages are separated by molts in which each stage-specific exoskeleton, or cuticle, is shed and replaced anew. Subtypes: positive regulation of nematode larval development [GO:0061063], negative regulation of nematode larval development [GO:0061064], regulation of dauer larval development [GO:0061065], regulation of nematode larval development, heterochronic [GO:0090444]